{
  "term_label": "actin filament-based movement",
  "gene": "UniProtKB:O43795",
  "term_id": "GO:0030048",
  "gene_name": "Unconventional myosin-Ib",
  "gene_symbol": "MYO1B"
}